{
  "term_id": "GO:0005102",
  "gene_name": "Amyloid-beta precursor protein",
  "gene_symbol": "APP",
  "gene": "UniProtKB:P05067",
  "term_label": "signaling receptor binding"
}